ectoine transmembrane transport [GO:0051470] (biological process) Definition: The directed movement of ectoine across a membrane by means of some agent such as a transporter or a pore. Ectoine (1,4,5,6-tetrahydro-2-methyl-4-pyrimidinecarboxylic acid) is a tetrahydropyrimidine commonly synthesized by halophilic bacteria. Relationships: is a type of monocarboxylic acid transport [GO:0015718]; is a type of GO:0071705; is a type of carboxylic acid transmembrane transport [GO:1905039] Also known as: ectoine transport Sources: GOC:ai